B-1b B cell differentiation [GO:0002338] (biological process) Sources: GOC:jal, ISBN:0781735149 Definition: The process in which B cells acquire the specialized features of B-1b B cells. B-1b B cells are B-1 cells that do not express CD5. Also known as: B-1b B lymphocyte differentiation, B-1b B-cell differentiation, B-1b B-lymphocyte differentiation, B-1b B cell development Note: Note that immunologists typically use the word 'development' to refer to cells of B or T cell lineages undergoing the process that GO describes as 'cell differentiation'. Relationships: is a type of B-1 B cell differentiation [GO:0001923]